{
  "gene_name": "Vitamin D-binding protein",
  "term_label": "vitamin D binding",
  "term_id": "GO:0005499",
  "gene_symbol": "GC",
  "gene": "UniProtKB:P02774"
}